carbamoyl-phosphate synthase (glutamine-hydrolyzing) activity [GO:0004088] (molecular function) Definition: Catalysis of the reaction: hydrogencarbonate + L-glutamine + 2 ATP + H2O = carbamoyl phosphate + L-glutamate + 2 ADP + phosphate + 2 H+. Sources: RHEA:18633 Also known as: carbamoyl phosphate synthase (glutamine-hydrolyzing) activity, CPS activity, GD-CPSase activity, carbamoyl phosphate synthetase activity, carbamoyl-phosphate synthase (glutamine-hydrolysing) activity, carbamoyl-phosphate synthetase (glutamine-hydrolysing) activity, carbamoyl-phosphate synthetase (glutamine-hydrolyzing) activity, carbamoylphosphate synthetase II activity, carbamyl phosphate synthetase (glutamine) activity, carbon-dioxide::L-glutamine amido-ligase (ADP-forming, carbamate-phosphorylating) activity, glutamine-dependent carbamoyl-phosphate synthase activity, glutamine-dependent carbamyl phosphate synthetase activity, hydrogen-carbonate:L-glutamine amido-ligase (ADP-forming, carbamate-phosphorylating) activity Relationships: is a type of GO:0016884